regulation of nuclear-transcribed mRNA catabolic process, deadenylation-dependent decay [GO:1900151] (biological process) Sources: GOC:TermGenie, GOC:mcc Also known as: regulation of deadenylation-dependent mRNA decay, regulation of mRNA breakdown, deadenylation-dependent decay, regulation of mRNA catabolic process, deadenylation-dependent, regulation of mRNA catabolic process, deadenylylation-dependent, regulation of mRNA catabolism, deadenylation-dependent, regulation of mRNA catabolism, deadenylylation-dependent, regulation of mRNA degradation, deadenylation-dependent decay, regulation of nuclear mRNA catabolic process, deadenylation-dependent decay Relationships: is a type of regulation of mRNA stability [GO:0043488]; regulates nuclear-transcribed mRNA catabolic process, deadenylation-dependent decay [GO:0000288] Definition: Any process that modulates the frequency, rate or extent of nuclear-transcribed mRNA catabolic process, deadenylation-dependent decay. Subtypes: GO:1900152, GO:1900153